{
  "gene": "UniProtKB:Q5IJ48",
  "term_label": "protein-containing complex",
  "gene_symbol": "CRB2",
  "gene_name": "Protein crumbs homolog 2",
  "term_id": "GO:0032991"
}